{
  "term_label": "nucleus",
  "gene": "UniProtKB:Q96MR9",
  "term_id": "GO:0005634",
  "gene_name": "Zinc finger protein 560",
  "gene_symbol": "ZNF560"
}